{
  "term_label": "G-protein beta/gamma-subunit complex binding",
  "term_id": "GO:0031683",
  "gene": "UniProtKB:P11488",
  "gene_name": "Guanine nucleotide-binding protein G(t) subunit alpha-1",
  "gene_symbol": "GNAT1"
}